viral envelope [GO:0019031] (cellular component) Definition: The lipid bilayer of a virion that surrounds the protein capsid. May also contain glycoproteins. Relationships: is a type of viral membrane [GO:0036338] Also known as: viral outside membrane, viral glycoprotein Sources: GOC:bf, GOC:bm, GOC:jl, ISBN:0781718325, Wikipedia:Viral_envelope